sodium-dependent multivitamin transmembrane transporter activity [GO:0008523] (molecular function) Relationships: is a type of GO:0015370; is a type of vitamin transmembrane transporter activity [GO:0090482] Sources: TC:2.A.21.5.2 Definition: Enables the transfer of a solute or solutes from one side of a membrane to the other according to the reaction: multivitamin(out) + Na+(out) = multivitamin(in) + Na+(in). Multivitamins include pantothenate, biotin and lipoate.